{
  "term_label": "cytokine activity",
  "term_id": "GO:0005125",
  "gene_symbol": "IFNA6",
  "gene": "UniProtKB:P05013",
  "gene_name": "Interferon alpha-6"
}